{
  "gene_symbol": "SLC24A3",
  "gene_name": "Sodium_potassium_calcium exchanger 3",
  "gene": "UniProtKB:Q9HC58",
  "term_id": "GO:0005262",
  "term_label": "calcium channel activity"
}